{
  "gene_name": "Integral membrane protein 2C",
  "term_label": "amyloid-beta binding",
  "gene": "UniProtKB:Q9NQX7",
  "term_id": "GO:0001540",
  "gene_symbol": "ITM2C"
}